laminin-5B complex [GO:0061801] (cellular component) Relationships: is a type of laminin complex [GO:0043256] Also known as: laminin 3B32 complex References: PMID:15979864 Sources: GOC:dph Definition: A laminin complex composed of alpha3B, beta3 and gamma2 polypeptide chains.